{
  "term_label": "Unknown molecular function",
  "gene_name": "Tripartite motif-containing protein 42",
  "gene": "UniProtKB:Q8IWZ5",
  "gene_symbol": "TRIM42",
  "term_id": "UNKNOWN:0001"
}